C5L2 anaphylatoxin chemotactic receptor binding [GO:0031715] (molecular function) Also known as: C5L2 anaphylatoxin chemotactic receptor ligand Relationships: is a type of GO:0031714 Sources: GOC:mah, GOC:nln Definition: Binding to a C5L2 anaphylatoxin chemotactic receptor.